N-acyltransferase activity [GO:0016410] (molecular function) Relationships: is a type of GO:0016747 Definition: Catalysis of the transfer of an acyl group to a nitrogen atom on the acceptor molecule. Subtypes: GO:0004379, N-acetyltransferase activity [GO:0008080], N-succinyltransferase activity [GO:0016749], peptidyl-lysine N6-palmitoyltransferase activity [GO:0018031], GO:0030270, GO:0043808, ornithine-acyl [acyl carrier protein] N-acyltransferase activity [GO:0043810], putrescine N-hydroxycinnamoyltransferase activity [GO:0047174], GO:0047946, glycine N-acyltransferase activity [GO:0047961], GO:0050291, isopenicillin-N N-acyltransferase activity [GO:0050640], N-malonyltransferase activity [GO:0050735], GO:0061579, protein propionyltransferase activity [GO:0061920], spermidine:sinapoyl CoA N-acyltransferase activity [GO:0080072], spermidine:coumaroyl CoA N-acyltransferase activity [GO:0080073], GO:0080074, GO:0080075, sinapoyl spermidine:sinapoyl CoA N-acyltransferase activity [GO:0080089], peptide N-succinyltransferase activity [GO:0106075], peptide 2-hydroxyisobutyryltransferase activity [GO:0106226], GO:0106228, peptide serotonyltransferase activity [GO:0120294], GO:0120296, GO:0120298, peptide histaminyltransferase activity [GO:0120299], GO:0120300, peptide crotonyltransferase activity [GO:0140064], GO:0140065, protein N-acyltransferase activity [GO:0140186] Sources: GOC:ai